brassinolide synthase activity [GO:0102734] (molecular function) Definition: Catalysis of the reaction: castasterone + O2 + reduced [NADPH--hemoprotein reductase] = brassinolide + H+ + H2O + oxidized [NADPH--hemoprotein reductase]. Broad specificity for several brassinosteroids, including castasterone, teasterone, and typhasterol. Sources: EC:1.14.14.180 Relationships: is a type of oxidoreductase activity, acting on paired donors, with incorporation or reduction of molecular oxygen, reduced flavin or flavoprotein as one donor, and incorporation of one atom of oxygen [GO:0016712]